{
  "term_id": "GO:0007165",
  "term_label": "signal transduction",
  "gene": "UniProtKB:Q8WYK1",
  "gene_symbol": "CNTNAP5",
  "gene_name": "Contactin-associated protein-like 5"
}